{
  "term_label": "Unknown biological process",
  "gene_symbol": "DMRTC1",
  "gene_name": "Doublesex- and mab-3-related transcription factor C1",
  "gene": "UniProtKB:Q5HYR2",
  "term_id": "UNKNOWN:0002"
}